hydroxydechloroatrazine ethylaminohydrolase activity [GO:0018763] (molecular function) Also known as: hydroxyatrazine ethylaminohydrolase activity, 4-(ethylamino)-2-hydroxy-6-(isopropylamino)-1,3,5-triazine ethylaminohydrolase activity, AtzB, hydroxyatrazine hydrolase activity Definition: Catalysis of the reaction: 4-(ethylamino)-2-hydroxy-6-(isopropylamino)-1,3,5-triazine + H2O = N-isopropylammelide + ethylamine. Sources: EC:3.5.4.43 Relationships: is a type of GO:0016810